{
  "term_id": "GO:0004843",
  "gene_symbol": "USP17L1",
  "gene": "UniProtKB:Q7RTZ2",
  "term_label": "cysteine-type deubiquitinase activity",
  "gene_name": "Ubiquitin carboxyl-terminal hydrolase 17-like protein 1"
}